{
  "term_id": "GO:0051082",
  "term_label": "unfolded protein binding",
  "gene": "UniProtKB:P49368",
  "gene_name": "T-complex protein 1 subunit gamma",
  "gene_symbol": "CCT3"
}